{
  "gene_symbol": "SLC35F5",
  "term_label": "Unknown cellular component",
  "term_id": "UNKNOWN:0003",
  "gene": "UniProtKB:Q8WV83",
  "gene_name": "Solute carrier family 35 member F5"
}